regulation of cellular response to amino acid starvation [GO:1903832] (biological process) References: PMID:25002487, PMID:7623840 Sources: GOC:TermGenie, GO_REF:0000058 Subtypes: negative regulation of cellular response to amino acid starvation [GO:1903574], positive regulation of cellular response to amino acid starvation [GO:1903833] Definition: Any process that modulates the frequency, rate or extent of cellular response to amino acid starvation. Relationships: is a type of regulation of response to nutrient levels [GO:0032107]; is a type of regulation of cellular response to stress [GO:0080135]; regulates cellular response to amino acid starvation [GO:0034198]